{
  "gene_symbol": "SPINK4",
  "term_label": "Unknown biological process",
  "gene": "UniProtKB:O60575",
  "term_id": "UNKNOWN:0002",
  "gene_name": "Serine protease inhibitor Kazal-type 4"
}